{
  "gene_symbol": "MVB12A",
  "gene_name": "Multivesicular body subunit 12A",
  "gene": "UniProtKB:Q96EY5",
  "term_id": "GO:0019075",
  "term_label": "virus maturation"
}